{
  "gene_name": "Putative small nuclear ribonucleoprotein G-like protein 15",
  "term_label": "U5 snRNP",
  "gene": "UniProtKB:A8MWD9",
  "gene_symbol": "SNRPGP15",
  "term_id": "GO:0005682"
}